{
  "gene_name": "Atos homolog protein A",
  "term_label": "Unknown biological process",
  "term_id": "UNKNOWN:0002",
  "gene": "UniProtKB:Q32MH5",
  "gene_symbol": "ATOSA"
}